{
  "gene": "UniProtKB:Q9Y3B8",
  "term_id": "UNKNOWN:0002",
  "gene_name": "Oligoribonuclease, mitochondrial",
  "gene_symbol": "REXO2",
  "term_label": "Unknown biological process"
}